{
  "term_id": "GO:0061630",
  "term_label": "ubiquitin protein ligase activity",
  "gene": "UniProtKB:O75677",
  "gene_name": "Ret finger protein-like 1",
  "gene_symbol": "RFPL1"
}